growth hormone-releasing hormone activity [GO:0016608] (molecular function) Also known as: GHRF activity, GHRH activity Sources: ISBN:0198506732 Definition: The action characteristic of growth hormone-releasing hormone, any of a family of peptide hormones that act on the anterior pituitary to stimulate the secretion of growth hormone and exert a trophic effect on the gland. Relationships: is a type of hormone activity [GO:0005179]